{
  "gene": "UniProtKB:A0A0U1RRE5",
  "term_id": "UNKNOWN:0001",
  "gene_symbol": "NBDY",
  "term_label": "Unknown molecular function",
  "gene_name": "Negative regulator of P-body association"
}